synaptic transmission, noradrenergic [GO:0099155] (BP) Relationships: is a type of GO:0007268 Definition: The vesicular release of noradrenaline (norepinephrine) a presynapse, across a chemical synapse, the subsequent activation of noradrenaline receptors at the postsynapse of a target cell (neuron, muscle, or secretory cell) and the effects of this activation on the postsynaptic membrane potential and ionic composition of the postsynaptic cytosol. This process encompasses both spontaneous and evoked release of neurotransmitter and all parts of synaptic vesicle exocytosis. Evoked transmission starts with the arrival of an action potential at the presynapse. Sources: GOC:dos, GOC:dph Also known as: noradrenergic synaptic transmission